aspartate kinase activity [GO:0004072] (molecular function) Also known as: ATP:L-aspartate 4-phosphotransferase activity, aspartic kinase activity, aspartokinase activity, beta-aspartokinase activity Relationships: is a type of phosphotransferase activity, carboxyl group as acceptor [GO:0016774]; is a type of amino acid kinase activity [GO:0019202] Sources: EC:2.7.2.4, RHEA:23776 Definition: Catalysis of the reaction: L-aspartate + ATP = 4-phospho-L-aspartate + ADP + H+.